{
  "gene_symbol": "DPH6",
  "term_id": "GO:0017183",
  "gene": "UniProtKB:Q7L8W6",
  "term_label": "protein histidyl modification to diphthamide",
  "gene_name": "Diphthine--ammonia ligase"
}